negative regulation of exocyst assembly [GO:0001929] (biological process) Also known as: down regulation of exocyst assembly, down-regulation of exocyst assembly, downregulation of exocyst assembly, inhibition of exocyst assembly Sources: GOC:hjd Definition: Any process that stops, prevents, or reduces the rate or extent of exocyst assembly. Relationships: is a type of GO:0001928; is a type of GO:0031333; is a type of negative regulation of exocytosis [GO:0045920]; RO_0002212 exocyst assembly [GO:0001927]